{
  "term_id": "GO:0051019",
  "gene_symbol": "MAPKAPK3",
  "term_label": "mitogen-activated protein kinase binding",
  "gene": "UniProtKB:Q16644",
  "gene_name": "MAP kinase-activated protein kinase 3"
}